{
  "term_label": "mediator complex",
  "term_id": "GO:0016592",
  "gene": "UniProtKB:Q6P2C8",
  "gene_symbol": "MED27",
  "gene_name": "Mediator of RNA polymerase II transcription subunit 27"
}